median body [GO:0097568] (cellular component) Note: Note that, due to the asymmetric nature of the Giardia trophozoite, this term is defined spatially as the trophozoite is viewed from the dorsal side, with the two nuclei dorsal to the ventral disc, and the ventral disc toward the anterior. Definition: A non-membrane bound, semi-organized microtubule array of unknown function found in Giardia species (trophozoite stage). It is located on the dorsal side of the trophozoite, slightly posterior to the ventral disc. References: PMID:5961344 Sources: GOC:giardia Also known as: parabasal body Relationships: is a type of GO:0110165; is part of GO:0005856; has part microtubule [GO:0005874]